regulation of early stripe melanocyte differentiation [GO:0050939] (biological process) Sources: GOC:ai Also known as: regulation of early stripe melanophore differentiation Relationships: is a type of regulation of melanocyte differentiation [GO:0045634]; regulates GO:0050933 Definition: Any process that modulates the frequency, rate or extent of early stripe melanocyte differentiation. Subtypes: GO:0050947, GO:0050948